{
  "gene": "UniProtKB:Q9UJA2",
  "gene_symbol": "CRLS1",
  "term_label": "cardiolipin synthase (CMP-forming)",
  "term_id": "GO:0043337",
  "gene_name": "Cardiolipin synthase (CMP-forming)"
}